{
  "gene_name": "S-adenosylhomocysteine hydrolase-like protein 1",
  "term_id": "GO:0005829",
  "gene": "UniProtKB:O43865",
  "gene_symbol": "AHCYL1",
  "term_label": "cytosol"
}